regulation of neuromuscular junction development [GO:1904396] (biological process) Also known as: regulation of neuromuscular junction organization, regulation of NMJ stability, regulation of neuromuscular junction stability References: PMID:7722643 Sources: GOC:TermGenie, GO_REF:0000058 Definition: Any process that modulates the frequency, rate or extent of neuromuscular junction development. Relationships: is a type of GO:0050807; regulates neuromuscular junction development [GO:0007528] Subtypes: regulation of synaptic assembly at neuromuscular junction [GO:0008582], negative regulation of neuromuscular junction development [GO:1904397], positive regulation of neuromuscular junction development [GO:1904398]